{
  "term_label": "cytoskeleton organization",
  "gene_symbol": "LIMD1",
  "term_id": "GO:0007010",
  "gene_name": "LIM domain-containing protein 1",
  "gene": "UniProtKB:Q9UGP4"
}